immune response-activating signaling pathway [GO:0002757] (biological process) Subtypes: immune response-activating cell surface receptor signaling pathway [GO:0002429], innate immune response-activating signaling pathway [GO:0002758] Definition: The series of molecular signals generated by a ligand binding to its receptor that lead to the activation or perpetuation of an immune response. Relationships: is a type of activation of immune response [GO:0002253]; is a type of GO:0002764 Sources: GOC:add Also known as: immune response-activating signal transduction